{
  "term_label": "neuropeptide Y receptor binding",
  "gene": "UniProtKB:Q5JQD4",
  "gene_symbol": "PYY3",
  "term_id": "GO:0031841",
  "gene_name": "Putative peptide YY-3"
}